{
  "gene": "UniProtKB:P61968",
  "term_label": "positive regulation of transcription by RNA polymerase II",
  "term_id": "GO:0045944",
  "gene_symbol": "LMO4",
  "gene_name": "LIM domain transcription factor LMO4"
}